monoterpene catabolic process [GO:0043694] (biological process) References: PMID:25076942 Subtypes: p-cymene catabolic process [GO:0019334], pinene catabolic process [GO:0033074], GO:0046251 Also known as: monoterpene catabolism Definition: The chemical reactions and pathways resulting in the breakdown of monoterpenes, terpenes with a C10 structure. Relationships: is a type of monoterpene metabolic process [GO:0043692]; is a type of GO:0046247